fusion of sperm to egg plasma membrane involved in single fertilization [GO:0007342] (biological process) References: PMID:17644969 Sources: GOC:dph, GOC:jl Relationships: is a type of cellular process involved in reproduction in multicellular organism [GO:0022412]; is_a plasma membrane fusion [GO:0045026]; is part of GO:0007338 Regulation: regulated by regulation of fusion of sperm to egg plasma membrane [GO:0043012]; negatively regulated by negative regulation of fusion of sperm to egg plasma membrane [GO:0043013] Definition: The binding and fusion of a sperm, with the plasma membrane of the oocyte as part of the process of single fertilization. In sperm with flagella, binding occurs at the posterior (post-acrosomal) region of the sperm head. Also known as: sperm-oocyte fusion